positive regulation of ventricular cardiac muscle cell action potential [GO:1903947] (biological process) Also known as: up regulation of ventricular cardiac muscle cell action potential, up-regulation of ventricular cardiac muscle cell action potential, upregulation of ventricular cardiac muscle cell action potential, activation of ventricular cardiac muscle cell action potential Definition: Any process that activates or increases the frequency, rate or extent of ventricular cardiac muscle cell action potential. References: PMID:25281747 Sources: GOC:BHF, GOC:TermGenie, GOC:mtg_cardiac_conduct_nov11, GOC:nc, GO_REF:0000058 Relationships: is a type of positive regulation of action potential [GO:0045760]; is a type of regulation of ventricular cardiac muscle cell action potential [GO:0098911]; is a type of positive regulation of cardiac muscle cell contraction [GO:0106134]; positively regulates ventricular cardiac muscle cell action potential [GO:0086005]